{
  "gene_symbol": "OR5B2",
  "gene_name": "Olfactory receptor 5B2",
  "term_id": "GO:0004984",
  "gene": "UniProtKB:Q96R09",
  "term_label": "olfactory receptor activity"
}